{
  "gene": "UniProtKB:Q6IEE8",
  "term_id": "UNKNOWN:0001",
  "gene_symbol": "SLFN12L",
  "term_label": "Unknown molecular function",
  "gene_name": "Schlafen family member 12-like"
}